{
  "term_label": "positive regulation of cytokine production involved in immune response",
  "gene_symbol": "TNFRSF14",
  "gene": "UniProtKB:Q92956",
  "term_id": "GO:0002720",
  "gene_name": "Tumor necrosis factor receptor superfamily member 14"
}